{
  "gene": "UniProtKB:P01569",
  "term_label": "B cell activation involved in immune response",
  "term_id": "GO:0002312",
  "gene_symbol": "IFNA5",
  "gene_name": "Interferon alpha-5"
}